{
  "gene_name": "Inhibitor of Bruton tyrosine kinase",
  "term_id": "GO:0005737",
  "gene": "UniProtKB:Q9P2D0",
  "term_label": "cytoplasm",
  "gene_symbol": "IBTK"
}